pyrrolizidine alkaloid biosynthetic process [GO:1901085] (biological process) Relationships: is a type of GO:0009821 Also known as: pyrrolizidine alkaloid anabolism, pyrrolizidine alkaloid biosynthesis, pyrrolizidine alkaloid formation, pyrrolizidine alkaloid synthesis References: PMID:30001795 Sources: GOC:TermGenie, GOC:yaf Definition: The chemical reactions and pathways resulting in the formation of pyrrolizidine alkaloid.